{
  "term_id": "GO:0007266",
  "gene_symbol": "CDC42EP2",
  "gene_name": "Cdc42 effector protein 2",
  "term_label": "Rho protein signal transduction",
  "gene": "UniProtKB:O14613"
}